{
  "gene_name": "LIM and senescent cell antigen-like-containing domain protein 4",
  "gene_symbol": "LIMS4",
  "term_label": "Unknown molecular function",
  "term_id": "UNKNOWN:0001",
  "gene": "UniProtKB:P0CW20"
}